{
  "gene_symbol": "HSFY2",
  "gene_name": "Heat shock transcription factor, Y-linked",
  "term_id": "GO:0000978",
  "term_label": "RNA polymerase II cis-regulatory region sequence-specific DNA binding",
  "gene": "UniProtKB:Q96LI6"
}